{
  "gene": "UniProtKB:Q8NBZ0",
  "gene_symbol": "INO80E",
  "term_id": "UNKNOWN:0002",
  "term_label": "Unknown biological process",
  "gene_name": "INO80 complex subunit E"
}